{
  "gene_name": "Hepatic triacylglycerol lipase",
  "gene_symbol": "LIPC",
  "gene": "UniProtKB:P11150",
  "term_id": "GO:0006633",
  "term_label": "fatty acid biosynthetic process"
}